{
  "gene": "UniProtKB:P51003",
  "gene_symbol": "PAPOLA",
  "term_label": "Unknown biological process",
  "gene_name": "Poly(A) polymerase alpha",
  "term_id": "UNKNOWN:0002"
}